{
  "term_label": "voltage-gated chloride channel activity",
  "gene_symbol": "CLCN5",
  "term_id": "GO:0005247",
  "gene": "UniProtKB:P51795",
  "gene_name": "H(+)_Cl(-) exchange transporter 5"
}